CD8-positive, alpha-beta regulatory T cell differentiation [GO:0002307] (biological process) Sources: GOC:add, ISBN:0781735149 Relationships: is a type of CD8-positive, alpha-beta T cell differentiation [GO:0043374]; is_a regulatory T cell differentiation [GO:0045066] Note: Note that immunologists typically use the word 'development' to refer to cells of B or T cell lineages undergoing the process that GO describes as 'cell differentiation'. Also known as: CD8-positive, alpha-beta regulatory T lymphocyte differentiation, CD8-positive, alpha-beta regulatory T-cell differentiation, CD8-positive, alpha-beta regulatory T-lymphocyte differentiation, CD8-positive, alpha-beta regulatory T cell development Definition: The process in which a precursor cell type acquires the specialized features of a CD8-positive, alpha-beta regulatory T cell.